regulation of macromolecule metabolic process [GO:0060255] (biological process) Definition: Any process that modulates the frequency, rate or extent of the chemical reactions and pathways involving macromolecules, any molecule of high relative molecular mass, the structure of which essentially comprises the multiple repetition of units derived, actually or conceptually, from molecules of low relative molecular mass. Relationships: is a type of GO:0019222; regulates macromolecule metabolic process [GO:0043170] Sources: GOC:dph, GOC:tb Subtypes: GO:0001919, GO:0010556, GO:0010604, negative regulation of macromolecule metabolic process [GO:0010605], regulation of cell wall macromolecule metabolic process [GO:0010981], regulation of polysaccharide metabolic process [GO:0032881], regulation of DNA metabolic process [GO:0051052], GO:0051246, regulation of RNA metabolic process [GO:0051252], regulation of phosphatidylinositol dephosphorylation [GO:0060304], regulation of receptor catabolic process [GO:2000644], GO:2000945